{
  "gene_symbol": "CCL18",
  "gene": "UniProtKB:P55774",
  "term_id": "GO:0008009",
  "term_label": "chemokine activity",
  "gene_name": "C-C motif chemokine 18"
}